{
  "term_label": "plasma membrane",
  "gene": "UniProtKB:A6NHS7",
  "gene_name": "MANSC domain-containing protein 4",
  "term_id": "GO:0005886",
  "gene_symbol": "MANSC4"
}